{
  "gene_symbol": "FNDC3B",
  "term_id": "UNKNOWN:0003",
  "term_label": "Unknown cellular component",
  "gene": "UniProtKB:Q53EP0",
  "gene_name": "Fibronectin type III domain-containing protein 3B"
}